{
  "gene": "UniProtKB:Q9H902",
  "term_label": "endoplasmic reticulum tubular network",
  "term_id": "GO:0071782",
  "gene_name": "Receptor expression-enhancing protein 1",
  "gene_symbol": "REEP1"
}